{
  "term_label": "nucleus",
  "gene": "UniProtKB:Q8IYR2",
  "gene_name": "SET and MYND domain-containing protein 4",
  "gene_symbol": "SMYD4",
  "term_id": "GO:0005634"
}